{
  "gene_name": "AP-1 complex subunit sigma-1A",
  "gene": "UniProtKB:P61966",
  "term_id": "UNKNOWN:0001",
  "term_label": "Unknown molecular function",
  "gene_symbol": "AP1S1"
}